triglyceride homeostasis [GO:0070328] (biological process) Subtypes: intracellular triglyceride homeostasis [GO:0035356] Definition: Any process involved in the maintenance of an internal steady state of triglyceride within an organism or cell. Sources: GOC:BHF, GOC:mah Also known as: triacylglycerol homeostasis Relationships: is a type of acylglycerol homeostasis [GO:0055090]